catechol oxidase activity [GO:0004097] (molecular function) Relationships: is a type of GO:0004497; is a type of oxidoreductase activity, acting on diphenols and related substances as donors, oxygen as acceptor [GO:0016682] Note: GO:0004097 describes oxidation of catechols (i.e., o-diphenols) to the corresponding o-quinones. For monooxygenation of monophenols, consider instead the term 'monophenol monooxygenase activity ; GO:0004503'. Also known as: phenolase activity, pyrocatechol oxidase, tyrosinase activity, catecholase, diphenol oxidase activity, o-diphenol oxidoreductase, o-diphenolase activity, L-DOPA monooxygenase activity, L-dopa oxidase activity, dopamine monooxygenase activity, polyphenol oxidase activity Definition: Catalysis of the reaction: 2 catechol + O2 = 2 1,2-benzoquinone + 2 H2O. This reaction catalyzes exclusively the oxidation of catechols (i.e., o-diphenols) to the corresponding o-quinones. References: PMID:22120533 Sources: EC:1.10.3.1